{
  "gene_symbol": "DNMBP",
  "term_id": "GO:0060271",
  "term_label": "cilium assembly",
  "gene_name": "Dynamin-binding protein",
  "gene": "UniProtKB:Q6XZF7"
}